{
  "gene_symbol": "ERP27",
  "term_label": "endoplasmic reticulum",
  "gene": "UniProtKB:Q96DN0",
  "gene_name": "Endoplasmic reticulum resident protein 27",
  "term_id": "GO:0005783"
}